negative regulation of FtsZ-dependent cytokinesis [GO:2000245] (BP) Also known as: negative regulation of prokaryote-type cytokinesis, negative regulation of prokaryotic fission Sources: GOC:mah Definition: Any process that stops, prevents, or reduces the frequency, rate or extent of Ftsz-dependent cytokinesis. Relationships: is a type of GO:0032466; is a type of GO:2000242; is a type of regulation of FtsZ-dependent cytokinesis [GO:2000244]; negatively regulates FtsZ-dependent cytokinesis [GO:0043093]